{
  "gene_name": "Large neutral amino acids transporter small subunit 1",
  "gene": "UniProtKB:Q01650",
  "term_id": "GO:0015804",
  "term_label": "neutral amino acid transport",
  "gene_symbol": "SLC7A5"
}